{
  "term_id": "GO:1904263",
  "term_label": "positive regulation of TORC1 signaling",
  "gene_symbol": "LAMTOR3",
  "gene": "UniProtKB:Q9UHA4",
  "gene_name": "Ragulator complex protein LAMTOR3"
}